{
  "gene": "UniProtKB:Q96NJ5",
  "term_label": "proteasome-mediated ubiquitin-dependent protein catabolic process",
  "term_id": "GO:0043161",
  "gene_symbol": "KLHL32",
  "gene_name": "Kelch-like protein 32"
}